{
  "gene_name": "Nucleoporin NUP188",
  "term_label": "nuclear pore inner ring",
  "gene_symbol": "NUP188",
  "gene": "UniProtKB:Q5SRE5",
  "term_id": "GO:0044611"
}